{
  "gene": "UniProtKB:Q86VQ3",
  "term_label": "Unknown molecular function",
  "gene_name": "Thioredoxin domain-containing protein 2",
  "gene_symbol": "TXNDC2",
  "term_id": "UNKNOWN:0001"
}